positive regulation of renal amino acid absorption [GO:1902754] (biological process) Relationships: is a type of positive regulation of multicellular organismal process [GO:0051240]; is a type of regulation of renal amino acid absorption [GO:1902752]; positively regulates renal amino acid absorption [GO:1990297] Also known as: up regulation of renal amino acid absorption, up-regulation of renal amino acid absorption, upregulation of renal amino acid absorption, activation of renal amino acid absorption References: PMID:1526373 Sources: GOC:TermGenie, GOC:hjd, GO_REF:0000058 Definition: Any process that activates or increases the frequency, rate or extent of renal amino acid absorption.